{
  "gene_name": "Vesicle transport through interaction with t-SNAREs homolog 1A",
  "gene_symbol": "VTI1A",
  "gene": "UniProtKB:Q96AJ9",
  "term_id": "GO:0005484",
  "term_label": "SNAP receptor activity"
}